{
  "gene_name": "Dual specificity protein phosphatase 8",
  "gene_symbol": "DUSP8",
  "term_id": "UNKNOWN:0002",
  "gene": "UniProtKB:Q13202",
  "term_label": "Unknown biological process"
}